{
  "gene": "UniProtKB:Q9BS86",
  "gene_symbol": "ZPBP",
  "gene_name": "Zona pellucida-binding protein 1",
  "term_id": "GO:0002199",
  "term_label": "zona pellucida receptor complex"
}